RNA (guanine-N7)-methylation [GO:0036265] (biological process) Relationships: is a type of RNA methylation [GO:0001510] Sources: GOC:BHF, GOC:rl Subtypes: rRNA (guanine-N7)-methylation [GO:0070476], tRNA (guanine-N7)-methylation [GO:0106004], GO:0106005 Definition: The addition of a methyl group to the N7 atom in the base portion of a guanine nucleotide residue in an RNA molecule.